positive regulation of phagocytosis [GO:0050766] (biological process) Subtypes: positive regulation of phagocytosis, engulfment [GO:0060100], positive regulation of opsonization [GO:1903028], GO:1905451, positive regulation of apoptotic cell clearance [GO:2000427] Relationships: is_a GO:0045807; is a type of GO:0050764; positively regulates phagocytosis [GO:0006909] Definition: Any process that activates or increases the frequency, rate or extent of phagocytosis. Also known as: up regulation of phagocytosis, up-regulation of phagocytosis, upregulation of phagocytosis, activation of phagocytosis, stimulation of phagocytosis Sources: GOC:ai